{
  "term_label": "positive regulation of hippo signaling",
  "gene": "UniProtKB:B3KU38",
  "gene_symbol": "IQCJ-SCHIP1",
  "term_id": "GO:0035332",
  "gene_name": "IQCJ-SCHIP1 readthrough transcript protein"
}